cellular detoxification of metal ion [GO:0140961] (biological process) Also known as: cellular detoxification of metal cation Subtypes: cellular detoxification of cadmium ion [GO:0098849], cellular detoxification of copper ion [GO:1990880] Relationships: is a type of GO:0061687; is a type of GO:1990748 References: PMID:26729300, PMID:33046888, PMID:34442707 Definition: Any process carried out at the cellular level that reduces or removes the toxicity of a metal ion.